{
  "gene_symbol": "SERPINE1",
  "term_id": "GO:0030195",
  "gene": "UniProtKB:P05121",
  "term_label": "negative regulation of blood coagulation",
  "gene_name": "Plasminogen activator inhibitor 1"
}